{
  "gene": "UniProtKB:Q9NX62",
  "term_id": "GO:0008254",
  "gene_name": "Golgi-resident adenosine 3',5'-bisphosphate 3'-phosphatase",
  "gene_symbol": "BPNT2",
  "term_label": "3'-nucleotidase activity"
}